{
  "term_label": "peptide hormone binding",
  "gene_name": "Growth hormone-releasing hormone receptor",
  "gene": "UniProtKB:Q02643",
  "gene_symbol": "GHRHR",
  "term_id": "GO:0017046"
}